metanephric proximal convoluted tubule segment 2 development [GO:0072232] (biological process) Definition: The process whose specific outcome is the progression of the S2 portion of the metanephric proximal convoluted tubule over time, from its formation to the mature structure. The S2 portion of the metanephric proximal tubule is involved in reabsorption of water and sodium chloride. Sources: GOC:bf, GOC:mtg_kidney_jan10 Also known as: metanephric S2 development Relationships: is a type of proximal convoluted tubule segment 2 development [GO:0072032]; is part of metanephric proximal convoluted tubule development [GO:0072229]